{
  "gene_symbol": "ATP1A1",
  "gene": "UniProtKB:P05023",
  "gene_name": "Sodium_potassium-transporting ATPase subunit alpha-1",
  "term_id": "GO:0036376",
  "term_label": "sodium ion export across plasma membrane"
}